{
  "term_label": "Unknown cellular component",
  "gene_symbol": "NR2F6",
  "gene": "UniProtKB:P10588",
  "gene_name": "Nuclear receptor subfamily 2 group F member 6",
  "term_id": "UNKNOWN:0003"
}